positive regulation of estrone secretion [GO:2000869] (biological process) Also known as: positive regulation of 3-hydroxy-1,3,5(10)-estratrien-17-one secretion, positive regulation of folliculin secretion Relationships: is a type of positive regulation of steroid hormone secretion [GO:2000833]; is_a regulation of estrone secretion [GO:2000867]; positively regulates estrone secretion [GO:0035943] Sources: GOC:sl Definition: Any process that activates or increases the frequency, rate or extent of estrone secretion.